mitotic intra-S DNA damage checkpoint signaling [GO:0031573] (biological process) Relationships: is a type of mitotic DNA damage checkpoint signaling [GO:0044773]; happens during mitotic S phase [GO:0000084] Sources: GOC:vw Also known as: S-phase checkpoint, intra-S DNA damage checkpoint, mitotic intra-S DNA damage checkpoint, signal transduction involved in intra-S DNA damage checkpoint Definition: A mitotic cell cycle checkpoint that slows DNA synthesis in response to DNA damage by the prevention of new origin firing and the stabilization of slow replication fork progression.